{
  "gene_name": "E3 ubiquitin-protein ligase MIB2",
  "term_label": "ubiquitin protein ligase activity",
  "gene": "UniProtKB:Q96AX9",
  "gene_symbol": "MIB2",
  "term_id": "GO:0061630"
}